oocyte axis specification [GO:0007309] (biological process) Relationships: is a type of developmental process involved in reproduction [GO:0003006]; is a type of axis specification [GO:0009798]; is part of GO:0007308 Sources: GOC:mtg_sensu, ISBN:0879694238 Also known as: oocyte axis determination Subtypes: GO:0007310, oocyte anterior/posterior axis specification [GO:0007314], oocyte animal/vegetal axis specification [GO:0060832] Definition: The establishment, maintenance and elaboration of an axis in the oocyte. An example of this is found in Drosophila melanogaster.